{
  "gene_symbol": "ZC2HC1A",
  "term_id": "UNKNOWN:0003",
  "term_label": "Unknown cellular component",
  "gene": "UniProtKB:Q96GY0",
  "gene_name": "Zinc finger C2HC domain-containing protein 1A"
}